{
  "gene_symbol": "ZBTB3",
  "term_label": "regulation of transcription by RNA polymerase II",
  "gene_name": "Zinc finger and BTB domain-containing protein 3",
  "term_id": "GO:0006357",
  "gene": "UniProtKB:Q9H5J0"
}